anaerobic electron transport chain [GO:0019645] (biological process) Relationships: is a type of respiratory electron transport chain [GO:0022904]; is part of anaerobic respiration [GO:0009061] Sources: GOC:ai, GOC:mtg_electron_transport Definition: A process in which a series of electron carriers operate together to transfer electrons from donors such as NADH and FADH2 to any of several different terminal electron acceptors other than oxygen to generate a transmembrane electrochemical gradient.